{
  "gene_symbol": "CGAS",
  "gene_name": "Cyclic GMP-AMP synthase",
  "gene": "UniProtKB:Q8N884",
  "term_label": "cytosol",
  "term_id": "GO:0005829"
}